TIR domain binding [GO:0070976] (molecular function) Also known as: Toll-Interleukin receptor domain binding Definition: Binding to a Toll-Interleukin receptor (TIR) domain of a protein. The TIR domain is an intracellular 200 residue domain that is found in the Toll protein, the interleukin-1 receptor (IL-1R), and MyD88; it contains three highly-conserved regions, and mediates protein-protein interactions between the Toll-like receptors (TLRs) and signal-transduction components. Sources: GOC:mah, InterPro:IPR000157 Relationships: is a type of GO:0019904